{
  "term_id": "UNKNOWN:0003",
  "gene": "UniProtKB:Q5T9C2",
  "gene_symbol": "EEIG1",
  "term_label": "Unknown cellular component",
  "gene_name": "Early estrogen-induced gene 1 protein"
}